cellular response to carbon monoxide [GO:0071245] (biological process) Sources: GOC:mah Definition: Any process that results in a change in state or activity of a cell (in terms of movement, secretion, enzyme production, gene expression, etc.) as a result of a carbon monoxide (CO) stimulus. Relationships: is a type of response to carbon monoxide [GO:0034465]; is a type of cellular response to oxygen-containing compound [GO:1901701]